[glutamine synthetase]-adenylyl-L-tyrosine phosphorylase activity [GO:0047388] (molecular function) Sources: RHEA:43716 Relationships: is a type of nucleotidyltransferase activity [GO:0016779]; is a type of catalytic activity, acting on a protein [GO:0140096] Also known as: adenylyl(glutamine synthetase) hydrolase activity, adenylyl-L-glutamate:ammonia ligase (ADP-forming) adenylylhydrolase activity, adenylyl-[glutamate-ammonia ligase] hydrolase activity, adenylyl-glutamate-ammonia ligase hydrolase activity, adenylyl-glutamine-synthetasehydrolase activity, [glutamine synthetase]-adenylyl-L-tyrosine phosphorylase Definition: Catalysis of the reaction: [glutamine synthetase]-O(4)-(5'-adenylyl)-L-tyrosine + phosphate = [glutamine synthetase]-L-tyrosine + ADP.